{
  "term_id": "GO:0035600",
  "gene_name": "Threonylcarbamoyladenosine tRNA methylthiotransferase",
  "term_label": "tRNA methylthiolation",
  "gene": "UniProtKB:Q5VV42",
  "gene_symbol": "CDKAL1"
}